{
  "gene_name": "[3-methyl-2-oxobutanoate dehydrogenase [lipoamide]] kinase, mitochondrial",
  "term_id": "GO:0010906",
  "term_label": "regulation of glucose metabolic process",
  "gene_symbol": "BCKDK",
  "gene": "UniProtKB:O14874"
}